{
  "gene_name": "Calmodulin-regulated spectrin-associated protein 3",
  "gene_symbol": "CAMSAP3",
  "term_id": "GO:0000076",
  "gene": "UniProtKB:Q9P1Y5",
  "term_label": "DNA replication checkpoint signaling"
}